{
  "gene_symbol": "PGK1",
  "gene": "UniProtKB:P00558",
  "term_id": "GO:0004618",
  "term_label": "phosphoglycerate kinase activity",
  "gene_name": "Phosphoglycerate kinase 1"
}